{
  "gene_symbol": "ARIH2",
  "term_label": "ubiquitin ligase complex",
  "gene_name": "E3 ubiquitin-protein ligase ARIH2",
  "term_id": "GO:0000151",
  "gene": "UniProtKB:O95376"
}